{
  "gene": "UniProtKB:Q13296",
  "gene_symbol": "SCGB2A2",
  "term_label": "Unknown molecular function",
  "gene_name": "Mammaglobin-A",
  "term_id": "UNKNOWN:0001"
}